{
  "term_label": "GTP binding",
  "gene_symbol": "GBP6",
  "gene": "UniProtKB:Q6ZN66",
  "gene_name": "Guanylate-binding protein 6",
  "term_id": "GO:0005525"
}